N-hydroxyarylamine O-acetyltransferase activity [GO:0046990] (molecular function) Definition: Catalysis of the reaction: acetyl-CoA + an N-hydroxyarylamine = CoA + an N-acetoxyarylamine. Sources: EC:2.3.1.118, MetaCyc:2.3.1.118-RXN Also known as: N-hydroxy-2-aminofluorene-O-acetyltransferase activity, acetyl-CoA:N-hydroxyarylamine O-acetyltransferase activity, arylhydroxamate N,O-acetyltransferase activity Relationships: is a type of O-acetyltransferase activity [GO:0016413]